{
  "gene": "UniProtKB:P54829",
  "term_id": "GO:0005829",
  "term_label": "cytosol",
  "gene_name": "Tyrosine-protein phosphatase non-receptor type 5",
  "gene_symbol": "PTPN5"
}